{
  "term_label": "regulation of amyloid precursor protein biosynthetic process",
  "term_id": "GO:0042984",
  "gene_symbol": "NECAB3",
  "gene": "UniProtKB:Q96P71",
  "gene_name": "N-terminal EF-hand calcium-binding protein 3"
}